{
  "gene": "UniProtKB:Q8N6N2",
  "gene_name": "Tetratricopeptide repeat protein 9B",
  "term_label": "Unknown molecular function",
  "gene_symbol": "TTC9B",
  "term_id": "UNKNOWN:0001"
}